{
  "gene": "UniProtKB:A0A0J9YVS3",
  "term_id": "UNKNOWN:0003",
  "gene_symbol": "IGHJ4",
  "gene_name": "Immunoglobulin heavy joining 4 (Fragment)",
  "term_label": "Unknown cellular component"
}